keratohyalin granule [GO:0036457] (CC) Relationships: is a type of cellular anatomical structure [GO:0110165]; is part of cytoplasm [GO:0005737] Definition: A cytoplasmic, non-membrane bound granule of, at least, keratinocyte. Associated to keratin intermediate filaments and partially crosslinked to the cell envelope. References: PMID:15854042 Sources: GOC:krc